{
  "term_id": "GO:0000978",
  "term_label": "RNA polymerase II cis-regulatory region sequence-specific DNA binding",
  "gene_name": "Zinc finger and SCAN domain-containing protein 23",
  "gene": "UniProtKB:Q3MJ62",
  "gene_symbol": "ZSCAN23"
}